{
  "term_id": "GO:0005794",
  "term_label": "Golgi apparatus",
  "gene": "UniProtKB:P52848",
  "gene_name": "Bifunctional heparan sulfate N-deacetylase_N-sulfotransferase 1",
  "gene_symbol": "NDST1"
}